{
  "term_label": "Unknown cellular component",
  "gene_name": "Putative uncharacterized protein LOC152225",
  "gene_symbol": "Q0VG73",
  "gene": "UniProtKB:Q0VG73",
  "term_id": "UNKNOWN:0003"
}